{
  "term_label": "stearoyl-CoA 9-desaturase activity",
  "gene_name": "Stearoyl-CoA desaturase 5",
  "gene": "UniProtKB:Q86SK9",
  "term_id": "GO:0004768",
  "gene_symbol": "SCD5"
}